cell morphogenesis [GO:0000902] (biological process) Also known as: cellular morphogenesis Definition: The developmental process in which the size or shape of a cell is generated and organized. Relationships: is a type of GO:0009653 Regulation: positively regulated by positive regulation of cell morphogenesis [GO:0010770]; negatively regulated by GO:0010771; regulated by regulation of cell morphogenesis [GO:0022604] Subtypes: cell morphogenesis involved in conjugation with cellular fusion [GO:0000753], inner cell mass cellular morphogenesis [GO:0001828], trophectodermal cellular morphogenesis [GO:0001831], epithelial cell morphogenesis [GO:0003382], histoblast morphogenesis [GO:0007488], unidimensional cell growth [GO:0009826], GO:0010090, trichome branching [GO:0010091], guard cell morphogenesis [GO:0010442], GO:0021943, follicle cell of egg chamber stalk formation [GO:0030713], platelet morphogenesis [GO:0036344], oocyte morphogenesis [GO:0048601], cell morphogenesis involved in neuron differentiation [GO:0048667], root hair initiation [GO:0048766], lateral line nerve glial cell morphogenesis involved in differentiation [GO:0048938], cell morphogenesis involved in semicircular canal fusion [GO:0060880], cell morphogenesis involved in Malpighian tubule morphogenesis [GO:0061336], lens fiber cell morphogenesis [GO:0070309], chondrocyte morphogenesis [GO:0090171], endothelial to hematopoietic transition [GO:0098508] Sources: GOC:clt, GOC:dph, GOC:go_curators, GOC:tb